positive regulation of voltage-gated calcium channel activity [GO:1901387] (BP) Subtypes: GO:1901843 Sources: GOC:BHF, GOC:TermGenie Relationships: is a type of regulation of voltage-gated calcium channel activity [GO:1901385]; is a type of positive regulation of cation channel activity [GO:2001259]; positively regulates voltage-gated calcium channel activity [GO:0005245] Also known as: activation of depolarization-activated calcium channel, positive regulation of depolarization-activated calcium channel, up regulation of depolarization-activated calcium channel, up-regulation of depolarization-activated calcium channel, upregulation of depolarization-activated calcium channel, activation of depolarization-activated voltage gated calcium channel activity, activation of depolarization-activated voltage-gated calcium channel, activation of depolarization-activated voltage-gated calcium channel activity, activation of voltage gated calcium channel activity, activation of voltage-dependent calcium channel activity, activation of voltage-gated calcium ion channel activity, activation of voltage-sensitive calcium channel, positive regulation of depolarization-activated voltage gated calcium channel activity, positive regulation of depolarization-activated voltage-gated calcium channel, positive regulation of depolarization-activated voltage-gated calcium channel activity, positive regulation of voltage gated calcium channel activity, positive regulation of voltage-dependent calcium channel activity, positive regulation of voltage-gated calcium ion channel activity, positive regulation of voltage-sensitive calcium channel, up regulation of depolarization-activated voltage gated calcium channel activity, up regulation of depolarization-activated voltage-gated calcium channel, up regulation of depolarization-activated voltage-gated calcium channel activity, up regulation of voltage gated calcium channel activity, up regulation of voltage-dependent calcium channel activity, up regulation of voltage-gated calcium channel activity, up regulation of voltage-gated calcium ion channel activity, up regulation of voltage-sensitive calcium channel, up-regulation of depolarization-activated voltage gated calcium channel activity, up-regulation of depolarization-activated voltage-gated calcium channel, up-regulation of depolarization-activated voltage-gated calcium channel activity, up-regulation of voltage gated calcium channel activity, up-regulation of voltage-dependent calcium channel activity, up-regulation of voltage-gated calcium channel activity, up-regulation of voltage-gated calcium ion channel activity, up-regulation of voltage-sensitive calcium channel, upregulation of depolarization-activated voltage gated calcium channel activity, upregulation of depolarization-activated voltage-gated calcium channel, upregulation of depolarization-activated voltage-gated calcium channel activity, upregulation of voltage gated calcium channel activity, upregulation of voltage-dependent calcium channel activity, upregulation of voltage-gated calcium channel activity, upregulation of voltage-gated calcium ion channel activity, upregulation of voltage-sensitive calcium channel, activation of dihydropyridine-sensitive calcium channel activity, activation of voltage-gated calcium channel activity, positive regulation of dihydropyridine-sensitive calcium channel activity, up regulation of dihydropyridine-sensitive calcium channel activity, up-regulation of dihydropyridine-sensitive calcium channel activity, upregulation of dihydropyridine-sensitive calcium channel activity Definition: Any process that activates or increases the frequency, rate or extent of voltage-gated calcium channel activity.